interferon-tau production [GO:0072651] (biological process) Also known as: IFN-tau production, IFN-tau secretion, IFNT production, interferon-tau secretion References: PMID:15546383 Sources: GOC:BHF, GOC:mah Note: Note that this term is in the subset of terms that should not be used for direct gene product annotation. Instead, select one of the 'regulation' children terms. Definition: The appearance of interferon-tau due to biosynthesis or secretion following a cellular stimulus, resulting in an increase in its intracellular or extracellular levels. Relationships: is a type of type I interferon production [GO:0032606]